dihydromethanopterin reductase activity [GO:0044684] (molecular function) Definition: Catalysis of the reaction: 7,8-dihydromethanopterin + NADPH = 5,6,7,8-tetrahydromethanopterin + NADP. Relationships: is_a oxidoreductase activity, acting on the CH-NH group of donors, NAD or NADP as acceptor [GO:0016646]; is part of tetrahydromethanopterin biosynthetic process [GO:2001118] References: PMID:15028691 Sources: GOC:mengo_curators